{
  "term_id": "UNKNOWN:0001",
  "gene_symbol": "ASPN",
  "term_label": "Unknown molecular function",
  "gene": "UniProtKB:Q9BXN1",
  "gene_name": "Asporin"
}